rhombomere 7 structural organization [GO:0021672] (biological process) Also known as: rhombomere 7 structural organisation Relationships: is a type of rhombomere structural organization [GO:0021595]; is part of rhombomere 7 morphogenesis [GO:0021671] Sources: GOC:cls, GOC:dgh, GOC:dph, GOC:jid, GO_REF:0000021 Definition: The process that contributes to creating the structural organization of rhombomere 7. This process pertains to the physical shaping of a rudimentary structure. Rhombomeres are transverse segments of the developing rhombencephalon. Rhombomeres are lineage restricted, express different genes from one another, and adopt different developmental fates. Rhombomeres are numbered in an anterior to posterior order.